{
  "term_label": "plasma membrane",
  "gene": "UniProtKB:Q8IYV9",
  "gene_name": "Izumo sperm-egg fusion protein 1",
  "gene_symbol": "IZUMO1",
  "term_id": "GO:0005886"
}